{
  "gene_symbol": "SERPINB1",
  "gene_name": "Leukocyte elastase inhibitor",
  "term_id": "GO:0005615",
  "term_label": "extracellular space",
  "gene": "UniProtKB:P30740"
}